{
  "gene_symbol": "SPP2",
  "gene": "UniProtKB:Q13103",
  "term_id": "UNKNOWN:0002",
  "term_label": "Unknown biological process",
  "gene_name": "Secreted phosphoprotein 24"
}